{
  "gene_name": "Ribose-phosphate pyrophosphokinase 1",
  "gene_symbol": "PRPS1",
  "gene": "UniProtKB:P60891",
  "term_id": "GO:0002189",
  "term_label": "ribose phosphate diphosphokinase complex"
}